N-terminal peptidyl-glutamic acid acetylation [GO:0018002] (biological process) Sources: RESID:AA0044 Relationships: is a type of N-terminal protein amino acid acetylation [GO:0006474]; is a type of GO:0018200 Definition: The acetylation of the N-terminal glutamic acid of proteins to form the derivate acetyl-glutamic acid. Note: See also the molecular function term 'aspartate N-acetyltransferase activity ; GO:0017188'.